germacrene A hydroxylase activity [GO:0106223] (molecular function) Relationships: is a type of GO:0016712 Definition: Catalysis of the reaction:(+)-(R)-germacrene A + 3 O2 + 3 reduced [NADPH--hemoprotein reductase] = germacra-1(10),4,11(13)-trien-12-oate + 4 H+ + 4 H2O + 3 oxidized [NADPH--hemoprotein reductase]. Also known as: germacrene A alcohol dehydrogenase activity References: PMID:11299372, PMID:20351109 Sources: RHEA:30303